{
  "gene_name": "Transient receptor potential cation channel subfamily M member 5",
  "term_id": "GO:0098655",
  "term_label": "monoatomic cation transmembrane transport",
  "gene_symbol": "TRPM5",
  "gene": "UniProtKB:Q9NZQ8"
}